AMP kinase activity [GO:0004017] (molecular function) Sources: RHEA:12973 Relationships: is_a nucleoside monophosphate kinase activity [GO:0050145] Also known as: adenylate kinase activity, myokinase activity, 5'-AMP-kinase activity, ATP:AMP phosphotransferase activity, adenylic kinase activity, adenylokinase activity Definition: Catalysis of the reaction: ATP + AMP = 2 ADP.